protein-N(PI)-phosphohistidine-sucrose phosphotransferase system transporter activity [GO:0022878] (molecular function) Sources: GOC:mtg_transport, ISBN:0815340729 Also known as: sucrose PTS transporter activity Definition: Catalysis of the PEP-dependent, phosphoryl transfer-driven transport of substances across a membrane. The transport happens by catalysis of the reaction: protein N-phosphohistidine + sucrose(out) = protein histidine + sucrose phosphate(in). This differs from primary and secondary active transport in that the solute is modified during transport. Relationships: is a type of sucrose transmembrane transporter activity [GO:0008515]; is a type of protein-N(PI)-phosphohistidine-sugar phosphotransferase activity [GO:0008982]